{
  "gene": "UniProtKB:Q6ZTR6",
  "gene_symbol": "ZNF516-DT",
  "term_label": "Unknown cellular component",
  "gene_name": "Putative uncharacterized protein ZNF516-DT",
  "term_id": "UNKNOWN:0003"
}